{
  "term_label": "N-acylphosphatidylethanolamine-specific phospholipase D activity",
  "term_id": "GO:0070290",
  "gene_symbol": "NAPEPLD",
  "gene_name": "N-acyl-phosphatidylethanolamine-hydrolyzing phospholipase D",
  "gene": "UniProtKB:Q6IQ20"
}